{
  "gene_name": "Angiopoietin-related protein 4",
  "term_id": "GO:0031012",
  "term_label": "extracellular matrix",
  "gene": "UniProtKB:Q9BY76",
  "gene_symbol": "ANGPTL4"
}